{
  "gene": "UniProtKB:P56177",
  "gene_name": "Homeobox protein DLX-1",
  "term_id": "GO:0000981",
  "gene_symbol": "DLX1",
  "term_label": "DNA-binding transcription factor activity, RNA polymerase II-specific"
}